{
  "gene_name": "Putative uncharacterized protein encoded by LINC01545",
  "gene_symbol": "LINC01545",
  "term_id": "UNKNOWN:0002",
  "term_label": "Unknown biological process",
  "gene": "UniProtKB:Q5VT33"
}